{
  "term_id": "GO:0009986",
  "gene": "UniProtKB:Q96JJ7",
  "gene_symbol": "TMX3",
  "term_label": "cell surface",
  "gene_name": "Protein disulfide-isomerase TMX3"
}